{
  "term_label": "Unknown biological process",
  "gene": "UniProtKB:A6NJ69",
  "gene_symbol": "IGIP",
  "gene_name": "IgA-inducing protein homolog",
  "term_id": "UNKNOWN:0002"
}